{
  "gene_symbol": "Q9UFV3",
  "term_id": "UNKNOWN:0002",
  "gene_name": "Putative uncharacterized protein DKFZp434L187",
  "gene": "UniProtKB:Q9UFV3",
  "term_label": "Unknown biological process"
}